{
  "gene_name": "ELAV-like protein 1",
  "gene_symbol": "ELAVL1",
  "term_label": "3'-UTR-mediated mRNA stabilization",
  "gene": "UniProtKB:Q15717",
  "term_id": "GO:0070935"
}